{
  "gene": "UniProtKB:Q8N0V4",
  "term_id": "GO:1904862",
  "term_label": "inhibitory synapse assembly",
  "gene_symbol": "LGI2",
  "gene_name": "Leucine-rich repeat LGI family member 2"
}